{
  "gene_symbol": "CRISP2",
  "term_id": "GO:0005615",
  "gene": "UniProtKB:P16562",
  "gene_name": "Cysteine-rich secretory protein 2",
  "term_label": "extracellular space"
}